positive regulation of chylomicron remnant clearance [GO:0090321] (biological process) Sources: GOC:BHF Definition: Any process that increases the rate, frequency or extent of chylomicron remnant clearance. Chylomicron clearance is the process in which a chylomicron remnant is removed from the blood via receptor-mediated endocytosis into liver cells and its constituent parts degraded. Relationships: is a type of GO:0010986; is a type of regulation of chylomicron remnant clearance [GO:0090320]; positively regulates chylomicron remnant clearance [GO:0034382]